{
  "gene_symbol": "PRR18",
  "term_id": "UNKNOWN:0001",
  "term_label": "Unknown molecular function",
  "gene": "UniProtKB:Q8N4B5",
  "gene_name": "Proline-rich protein 18"
}